eggshell chorion gene amplification [GO:0007307] (biological process) References: PMID:11157771 Sources: GOC:mtg_sensu Relationships: is a type of GO:0006277; is a type of cellular process involved in reproduction in multicellular organism [GO:0022412]; is part of egg chorion assembly [GO:0007306] Definition: Amplification by up to 60-fold of the loci containing the chorion gene clusters. Amplification is necessary for the rapid synthesis of chorion proteins by the follicle cells, and occurs by repeated firing of one or more origins located within each gene cluster.